trigeminal nerve structural organization [GO:0021637] (BP) Also known as: trigeminal nerve structural organisation, CN V structural organization Relationships: is a type of cranial nerve structural organization [GO:0021604]; BFO_0000050 GO:0021636 Sources: GOC:cls, GOC:dgh, GOC:dph, GOC:jid, GO_REF:0000021 Definition: The process that contributes to the act of creating the structural organization of the oculomotor nerve. This process pertains to the physical shaping of a rudimentary structure. The trigeminal nerve is composed of three large branches. They are the ophthalmic (V1, sensory), maxillary (V2, sensory) and mandibular (V3, motor and sensory) branches. The sensory ophthalmic branch travels through the superior orbital fissure and passes through the orbit to reach the skin of the forehead and top of the head. The maxillary nerve contains sensory branches that reach the pterygopalatine fossa via the inferior orbital fissure (face, cheek and upper teeth) and pterygopalatine canal (soft and hard palate, nasal cavity and pharynx). The motor part of the mandibular branch is distributed to the muscles of mastication, the mylohyoid muscle and the anterior belly of the digastric. The mandibular nerve also innervates the tensor veli palatini and tensor tympani muscles. The sensory part of the mandibular nerve is composed of branches that carry general sensory information from the mucous membranes of the mouth and cheek, anterior two-thirds of the tongue, lower teeth, skin of the lower jaw, side of the head and scalp and meninges of the anterior and middle cranial fossae.